{
  "term_label": "macrophage migration inhibitory factor binding",
  "term_id": "GO:0035718",
  "gene": "UniProtKB:P04233",
  "gene_symbol": "CD74",
  "gene_name": "HLA class II histocompatibility antigen gamma chain"
}